regulation of convergent extension involved in somitogenesis [GO:1904127] (biological process) References: PMID:24892953 Sources: GOC:TermGenie, GOC:dph, GO_REF:0000058 Subtypes: negative regulation of convergent extension involved in somitogenesis [GO:1904128], positive regulation of convergent extension involved in somitogenesis [GO:1904129] Relationships: is a type of regulation of convergent extension involved in axis elongation [GO:1901232]; is a type of regulation of convergent extension involved in gastrulation [GO:1904103]; regulates convergent extension involved in somitogenesis [GO:0090246] Definition: Any process that modulates the frequency, rate or extent of convergent extension involved in somitogenesis.